{
  "term_id": "GO:0032050",
  "gene_name": "Clathrin light chain B",
  "term_label": "clathrin heavy chain binding",
  "gene": "UniProtKB:P09497",
  "gene_symbol": "CLTB"
}